{
  "gene_symbol": "CCDC169",
  "gene": "UniProtKB:A6NNP5",
  "term_label": "Unknown cellular component",
  "gene_name": "Coiled-coil domain-containing protein 169",
  "term_id": "UNKNOWN:0003"
}